{
  "gene_name": "Chromosome-associated kinesin KIF4A",
  "term_label": "microtubule motor activity",
  "gene_symbol": "KIF4A",
  "term_id": "GO:0003777",
  "gene": "UniProtKB:O95239"
}